{
  "term_label": "positive regulation of cell population proliferation",
  "term_id": "GO:0008284",
  "gene_name": "GTPase KRas",
  "gene": "UniProtKB:P01116",
  "gene_symbol": "KRAS"
}